positive regulation of calcium ion-dependent exocytosis [GO:0045956] (biological process) Relationships: is a type of GO:0017158; is_a positive regulation of regulated secretory pathway [GO:1903307]; positively regulates calcium-ion regulated exocytosis [GO:0017156] Subtypes: positive regulation of cortical granule exocytosis by positive regulation of cytosolic calcium ion concentration [GO:0060472], GO:1903235, positive regulation of dense core granule exocytosis [GO:1905415], GO:2000368 Sources: GOC:go_curators Also known as: up regulation of calcium ion-dependent exocytosis, up-regulation of calcium ion-dependent exocytosis, upregulation of calcium ion-dependent exocytosis, activation of calcium ion-dependent exocytosis, stimulation of calcium ion-dependent exocytosis Definition: Any process that activates or increases the frequency, rate or extent of calcium ion-dependent exocytosis.